{
  "gene_symbol": "RNF38",
  "term_id": "GO:0016567",
  "gene_name": "E3 ubiquitin-protein ligase RNF38",
  "term_label": "protein ubiquitination",
  "gene": "UniProtKB:Q9H0F5"
}